8-demethylnovobiocate synthase activity [GO:0102527] (molecular function) Sources: EC:6.3.1.15, GOC:pz Definition: Catalysis of the reaction: 3-amino-4,7-dihydroxycoumarin + 3-dimethylallyl-4-hydroxybenzoate + ATP(4-) = H+ + 8-desmethylnovobiocic acid(1-) + AMP(2-) + diphosphoric acid. Relationships: is a type of acid-ammonia (or amide) ligase activity [GO:0016880]